negative regulation of response to ethanol [GO:1901417] (biological process) Also known as: down regulation of response to ethanol, down-regulation of response to ethanol, downregulation of response to ethanol, inhibition of response to ethanol Relationships: is a type of regulation of response to ethanol [GO:1901416]; is a type of negative regulation of response to alcohol [GO:1901420]; negatively regulates response to ethanol [GO:0045471] Sources: GOC:TermGenie, GOC:mengo_curators Definition: Any process that stops, prevents or reduces the frequency, rate or extent of response to ethanol.